{
  "gene_symbol": "CYP2D7",
  "term_label": "xenobiotic metabolic process",
  "gene_name": "Putative cytochrome P450 2D7",
  "gene": "UniProtKB:A0A087X1C5",
  "term_id": "GO:0006805"
}